{
  "gene_name": "Transcobalamin-2",
  "term_label": "cobalamin binding",
  "gene": "UniProtKB:P20062",
  "gene_symbol": "TCN2",
  "term_id": "GO:0031419"
}